{
  "gene_symbol": "ADHFE1",
  "gene_name": "Hydroxyacid-oxoacid transhydrogenase, mitochondrial",
  "term_label": "Unknown biological process",
  "term_id": "UNKNOWN:0002",
  "gene": "UniProtKB:Q8IWW8"
}